{
  "term_label": "nucleus",
  "term_id": "GO:0005634",
  "gene_symbol": "NYNRIN",
  "gene_name": "Protein NYNRIN",
  "gene": "UniProtKB:Q9P2P1"
}